{
  "gene_symbol": "MNAT1",
  "term_label": "transcription factor TFIIH holo complex",
  "gene": "UniProtKB:P51948",
  "term_id": "GO:0005675",
  "gene_name": "CDK-activating kinase assembly factor MAT1"
}